{
  "gene_symbol": "OR4C45",
  "term_id": "UNKNOWN:0002",
  "term_label": "Unknown biological process",
  "gene": "UniProtKB:A6NMZ5",
  "gene_name": "Olfactory receptor 4C45"
}